positive regulation of DNA strand resection involved in replication fork processing [GO:0106253] (biological process) Definition: Any process that activates or increases the frequency, rate or extent of DNA strand resection involved in replication fork processing. References: PMID:31575705 Sources: GOC:vw Relationships: is a type of positive regulation of DNA metabolic process [GO:0051054]; is a type of regulation of DNA strand resection involved in replication fork processing [GO:0110026]; positively regulates GO:0110025